{
  "term_id": "GO:0010976",
  "gene": "UniProtKB:Q14162",
  "gene_symbol": "SCARF1",
  "gene_name": "Scavenger receptor class F member 1",
  "term_label": "positive regulation of neuron projection development"
}